positive regulation of (Z)-nonadeca-1,14-diene biosynthetic process [GO:1900943] (biological process) Relationships: is a type of positive regulation of olefin biosynthetic process [GO:1900913]; is a type of regulation of (Z)-nonadeca-1,14-diene biosynthetic process [GO:1900941]; positively regulates GO:1900879 Also known as: positive regulation of (Z)-nonadeca-1,14-diene anabolism, positive regulation of (Z)-nonadeca-1,14-diene biosynthesis, positive regulation of (Z)-nonadeca-1,14-diene formation, positive regulation of (Z)-nonadeca-1,14-diene synthesis, up regulation of (Z)-nonadeca-1,14-diene anabolism, up regulation of (Z)-nonadeca-1,14-diene biosynthesis, up regulation of (Z)-nonadeca-1,14-diene biosynthetic process, up regulation of (Z)-nonadeca-1,14-diene formation, up regulation of (Z)-nonadeca-1,14-diene synthesis, up-regulation of (Z)-nonadeca-1,14-diene anabolism, up-regulation of (Z)-nonadeca-1,14-diene biosynthesis, up-regulation of (Z)-nonadeca-1,14-diene biosynthetic process, up-regulation of (Z)-nonadeca-1,14-diene formation, up-regulation of (Z)-nonadeca-1,14-diene synthesis, upregulation of (Z)-nonadeca-1,14-diene anabolism, upregulation of (Z)-nonadeca-1,14-diene biosynthesis, upregulation of (Z)-nonadeca-1,14-diene biosynthetic process, upregulation of (Z)-nonadeca-1,14-diene formation, upregulation of (Z)-nonadeca-1,14-diene synthesis, activation of (Z)-nonadeca-1,14-diene anabolism, activation of (Z)-nonadeca-1,14-diene biosynthesis, activation of (Z)-nonadeca-1,14-diene biosynthetic process, activation of (Z)-nonadeca-1,14-diene formation, activation of (Z)-nonadeca-1,14-diene synthesis Sources: GOC:TermGenie, GOC:mengo_curators Definition: Any process that activates or increases the frequency, rate or extent of (Z)-nonadeca-1,14-diene biosynthetic process.